cichorine biosynthetic process [GO:0062032] (biological process) Definition: The chemical reactions and pathways resulting in the formation of cichorine, a secondary metabolite found in some species of fungi. Relationships: is a type of secondary metabolite biosynthetic process [GO:0044550]; is a type of phenol-containing compound biosynthetic process [GO:0046189] Also known as: cichorine anabolism, cichorine biosynthesis, cichorine formation, cichorine synthesis References: PMID:24244835